{
  "term_id": "GO:0008020",
  "gene": "UniProtKB:P47804",
  "gene_symbol": "RGR",
  "gene_name": "RPE-retinal G protein-coupled receptor",
  "term_label": "G protein-coupled photoreceptor activity"
}